{
  "gene_symbol": "NCBP1",
  "gene_name": "Nuclear cap-binding protein subunit 1",
  "gene": "UniProtKB:Q09161",
  "term_id": "GO:0000339",
  "term_label": "RNA cap binding"
}